{
  "gene_symbol": "MRPS34",
  "term_id": "GO:0005763",
  "gene": "UniProtKB:P82930",
  "gene_name": "Small ribosomal subunit protein mS34",
  "term_label": "mitochondrial small ribosomal subunit"
}